metanephric cortical collecting duct development [GO:0072219] (BP) Definition: The process whose specific outcome is the progression of the metanephric cortical collecting duct over time, from its formation to the mature structure. The metanephric cortical collecting duct is the portion of the metanephric collecting duct that resides in the renal cortex. Relationships: is a type of cortical collecting duct development [GO:0072059] Sources: GOC:mtg_kidney_jan10